{
  "gene": "UniProtKB:Q02643",
  "gene_name": "Growth hormone-releasing hormone receptor",
  "term_id": "GO:0005886",
  "gene_symbol": "GHRHR",
  "term_label": "plasma membrane"
}